{
  "gene_name": "Choline_ethanolamine kinase",
  "term_label": "CDP-choline pathway",
  "gene_symbol": "CHKB",
  "gene": "UniProtKB:Q9Y259",
  "term_id": "GO:0006657"
}